calmodulin-activated dual specificity 3',5'-cyclic-GMP, 3',5'-cyclic-AMP phosphodiesterase activity [GO:0004117] (molecular function) Relationships: is a type of 3',5'-cyclic-AMP phosphodiesterase activity [GO:0004115]; is a type of 3',5'-cyclic-GMP phosphodiesterase activity [GO:0047555] References: PMID:8557689, PMID:9419816 Also known as: calmodulin-dependent cyclic-nucleotide phosphodiesterase activity, calmodulin-activated cyclic-nucleotide dual specificity phosphodiesterase activity Definition: Catalysis of the reactions: 3',5'-cyclic AMP + H2O = AMP + H+ and 3',5'-cyclic GMP + H2O = GMP + H+; this activity is activated by binding to calcium-bound calmodulin.